{
  "term_id": "UNKNOWN:0002",
  "gene_symbol": "PPWD1",
  "term_label": "Unknown biological process",
  "gene_name": "Peptidylprolyl isomerase domain and WD repeat-containing protein 1",
  "gene": "UniProtKB:Q96BP3"
}